neurohypophyseal hormone activity [GO:0005185] (molecular function) Also known as: neurohypophysial hormone activity Definition: The action characteristic of a neurohypophyseal hormone, any of a family of structurally and functionally related nonapeptides that are synthesized as part of a larger precursor molecule comprising a signal peptide, the nonapeptide hormone, and a neurophysin. Relationships: is a type of neuropeptide hormone activity [GO:0005184] References: PMID:19243634 Sources: GOC:mah